apolipoprotein E recycling [GO:0071828] (biological process) Also known as: APOE recycling Relationships: is a type of protein transport [GO:0015031]; is part of high-density lipoprotein particle assembly [GO:0034380]; is part of chylomicron remnant clearance [GO:0034382] References: PMID:16373604 Sources: GOC:BHF Definition: The process in which chylomicron remnant-associated apolipoprotein E is internalized by endocytosis, localized to recycling endosomes and then secreted in association with a high-density lipoprotein particle.